{
  "gene_symbol": "TMC5",
  "gene_name": "Transmembrane channel-like protein 5",
  "term_label": "Unknown biological process",
  "gene": "UniProtKB:Q6UXY8",
  "term_id": "UNKNOWN:0002"
}